{
  "gene": "UniProtKB:A6NI79",
  "gene_name": "Coiled-coil domain-containing protein 69",
  "term_label": "Unknown biological process",
  "term_id": "UNKNOWN:0002",
  "gene_symbol": "CCDC69"
}